{
  "gene": "UniProtKB:Q8WW36",
  "gene_symbol": "ZCCHC13",
  "term_id": "GO:0005737",
  "term_label": "cytoplasm",
  "gene_name": "Zinc finger CCHC domain-containing protein 13"
}